{
  "term_id": "GO:0005125",
  "term_label": "cytokine activity",
  "gene_symbol": "IL19",
  "gene_name": "Interleukin-19",
  "gene": "UniProtKB:Q9UHD0"
}